{
  "gene_symbol": "PIM1",
  "term_id": "GO:0043066",
  "gene": "UniProtKB:P11309",
  "gene_name": "Serine_threonine-protein kinase pim-1",
  "term_label": "negative regulation of apoptotic process"
}